{
  "term_label": "extracellular matrix organization",
  "gene": "UniProtKB:Q9UEW3",
  "gene_symbol": "MARCO",
  "term_id": "GO:0030198",
  "gene_name": "Macrophage receptor MARCO"
}